thyroid gland epithelial cell proliferation [GO:1990789] (biological process) References: PMID:17646383 Relationships: is_a epithelial cell proliferation [GO:0050673]; BFO_0000050 GO:0030878 Regulation: regulated by regulation of thyroid gland epithelial cell proliferation [GO:1904441]; negatively regulated by negative regulation of thyroid gland epithelial cell proliferation [GO:1904442]; positively regulated by positive regulation of thyroid gland epithelial cell proliferation [GO:1904443] Also known as: Hurthle cell proliferation, thyroid follicular cell proliferation Definition: The multiplication or reproduction of thyroid gland epithelial cells, resulting in the expansion of the thyroid gland epithelial cell population.